{
  "gene_symbol": "FBXW4",
  "gene": "UniProtKB:P57775",
  "term_id": "GO:0019005",
  "term_label": "SCF ubiquitin ligase complex",
  "gene_name": "F-box_WD repeat-containing protein 4"
}